{
  "gene_name": "Centrin-2",
  "term_label": "nucleus",
  "gene": "UniProtKB:P41208",
  "gene_symbol": "CETN2",
  "term_id": "GO:0005634"
}